peptidyl-serine modification [GO:0018209] (biological process) Relationships: is a type of peptidyl-amino acid modification [GO:0018193] Subtypes: peptidyl-serine phosphopantetheinylation [GO:0018070], peptidyl-L-3-oxoalanine biosynthetic process from peptidyl-cysteine or peptidyl-serine [GO:0018083], peptidyl-serine phosphorylation [GO:0018105], peptidyl-serine octanoylation [GO:0018191], protein-phosphoribosyl dephospho-coenzyme A linkage [GO:0018247], RNA-protein covalent cross-linking via peptidyl-serine [GO:0018259], peptidyl-serine O-acetylation [GO:0030919], GO:0035570 Definition: The modification of peptidyl-serine. Sources: GOC:go_curators